{
  "gene": "UniProtKB:P60409",
  "term_id": "UNKNOWN:0001",
  "term_label": "Unknown molecular function",
  "gene_symbol": "KRTAP10-7",
  "gene_name": "Keratin-associated protein 10-7"
}